{
  "gene_symbol": "SEMA4B",
  "term_id": "GO:0005886",
  "term_label": "plasma membrane",
  "gene_name": "Semaphorin-4B",
  "gene": "UniProtKB:Q9NPR2"
}